regulation of bacterial-type flagellum assembly [GO:1902208] (biological process) Definition: Any process that modulates the frequency, rate or extent of bacterial-type flagellum assembly. Sources: GOC:TermGenie, GOC:jl Also known as: regulation of bacterial flagellum assembly Relationships: is a type of regulation of cell projection assembly [GO:0060491]; is a type of regulation of organelle assembly [GO:1902115]; regulates bacterial-type flagellum assembly [GO:0044780] Subtypes: negative regulation of bacterial-type flagellum assembly [GO:1902209], GO:1902210